{
  "gene_symbol": "ARFGAP2",
  "gene_name": "ADP-ribosylation factor GTPase-activating protein 2",
  "term_label": "Unknown cellular component",
  "gene": "UniProtKB:Q8N6H7",
  "term_id": "UNKNOWN:0003"
}